{
  "gene": "UniProtKB:P84243",
  "term_id": "GO:0051382",
  "term_label": "kinetochore assembly",
  "gene_name": "Histone H3.3",
  "gene_symbol": "H3-3B"
}